{
  "term_id": "GO:0050211",
  "gene": "UniProtKB:Q8NBJ5",
  "term_label": "procollagen galactosyltransferase activity",
  "gene_name": "Procollagen galactosyltransferase 1",
  "gene_symbol": "COLGALT1"
}